{
  "gene_symbol": "PECAM1",
  "term_id": "GO:0009897",
  "gene_name": "Platelet endothelial cell adhesion molecule",
  "term_label": "external side of plasma membrane",
  "gene": "UniProtKB:P16284"
}